{
  "gene_symbol": "RAB3GAP2",
  "term_label": "synaptic signaling",
  "term_id": "GO:0099536",
  "gene": "UniProtKB:Q9H2M9",
  "gene_name": "Rab3 GTPase-activating protein non-catalytic subunit"
}